{
  "gene": "UniProtKB:Q5T7W7",
  "term_label": "Unknown cellular component",
  "gene_symbol": "TSTD2",
  "term_id": "UNKNOWN:0003",
  "gene_name": "Thiosulfate sulfurtransferase_rhodanese-like domain-containing protein 2"
}